{
  "gene_name": "Homeobox protein Hox-B9",
  "gene_symbol": "HOXB9",
  "gene": "UniProtKB:P17482",
  "term_id": "GO:0003700",
  "term_label": "DNA-binding transcription factor activity"
}